xanthophyll catabolic process [GO:0016124] (BP) Relationships: is a type of carotenoid catabolic process [GO:0016118]; is a type of xanthophyll metabolic process [GO:0016122] Definition: The chemical reactions and pathways resulting in the breakdown of xanthophylls, oxygen-containing carotenoids. Subtypes: rhodopsin catabolic process [GO:0046155], GO:0062172, GO:1901179, capsanthin catabolic process [GO:1901808], GO:1901814, zeaxanthin catabolic process [GO:1901826], all-trans-neoxanthin catabolic process [GO:1901832], GO:1901865 Sources: GOC:go_curators Also known as: xanthophyll breakdown, xanthophyll catabolism, xanthophyll degradation